response to mercaptoethanol [GO:0072704] (BP) Definition: Any process that results in a change in state or activity of a cell or an organism (in terms of movement, secretion, enzyme production, gene expression, etc.) as a result of a mercaptoethanol stimulus. Sources: GOC:mah Also known as: response to 2-sulfanylethanol Relationships: is a type of response to alcohol [GO:0097305] Subtypes: cellular response to mercaptoethanol [GO:0072705]